{
  "term_id": "GO:0019005",
  "gene": "UniProtKB:Q9UKA1",
  "gene_symbol": "FBXL5",
  "term_label": "SCF ubiquitin ligase complex",
  "gene_name": "F-box_LRR-repeat protein 5"
}